{
  "gene_symbol": "PVR",
  "gene_name": "Poliovirus receptor",
  "term_label": "heterophilic cell-cell adhesion",
  "term_id": "GO:0007157",
  "gene": "UniProtKB:P15151"
}